regulation of vascular associated smooth muscle cell membrane depolarization [GO:1990736] (biological process) Also known as: regulation of vascular smooth muscle cell membrane depolarization Relationships: is a type of membrane depolarization [GO:0051899] Definition: Any process that modulates the establishment or extent of a membrane potential in the depolarizing direction away from the resting potential in a vascular smooth muscle cell. Regulation: negatively regulated by negative regulation of regulation of vascular associated smooth muscle cell membrane depolarization [GO:1904198]; positively regulated by GO:1904199 References: PMID:20826763